{
  "gene": "UniProtKB:P52789",
  "gene_name": "Hexokinase-2",
  "gene_symbol": "HK2",
  "term_id": "GO:0005829",
  "term_label": "cytosol"
}